{
  "term_label": "DNA-binding transcription factor activity, RNA polymerase II-specific",
  "gene_name": "Transcriptional repressor scratch 1",
  "gene_symbol": "SCRT1",
  "term_id": "GO:0000981",
  "gene": "UniProtKB:Q9BWW7"
}